{
  "term_id": "GO:0051963",
  "gene": "UniProtKB:Q9P121",
  "gene_name": "Neurotrimin",
  "term_label": "regulation of synapse assembly",
  "gene_symbol": "NTM"
}